high-affinity sulfate:proton symporter activity [GO:0009675] (molecular function) Relationships: is a type of GO:0008512 Sources: GOC:mah Definition: Enables the transfer of a solute or solutes from one side of a membrane to the other according to the reaction: sulfate(out) + H+(out) = sulfate(in) + H+(in). In high-affinity transport the transporter is able to bind the solute even if it is only present at very low concentrations. Also known as: high affinity sulfate:hydrogen symporter activity, high affinity sulfate:proton symporter activity, high affinity sulphate:hydrogen symporter activity